{
  "term_id": "UNKNOWN:0001",
  "gene_name": "NADH dehydrogenase [ubiquinone] iron-sulfur protein 5",
  "term_label": "Unknown molecular function",
  "gene": "UniProtKB:O43920",
  "gene_symbol": "NDUFS5"
}